{
  "gene": "UniProtKB:P01764",
  "term_id": "GO:0016064",
  "term_label": "immunoglobulin mediated immune response",
  "gene_symbol": "IGHV3-23",
  "gene_name": "Immunoglobulin heavy variable 3-23"
}